establishment of turgor in appressorium [GO:0075039] (biological process) Note: Note that this term should not be used to annotate gene products of the host. It should only be used to annotate those gene products from the symbiont involved in this process. Also known as: establishment of turgor in symbiont appressorium on or near host, formation of turgor in appressorium, generation of turgor in appressorium Relationships: is a type of formation of structure involved in a symbiotic process [GO:0044111]; is part of appressorium maturation [GO:0075035] Sources: GOC:pamgo_curators Definition: The process in which hydrostatic pressure is increased within the symbiont appressorium to breach the cuticle of the host. The host is defined as the larger of the organisms involved in a symbiotic interaction.